regulation of wax biosynthetic process [GO:1904276] (biological process) Definition: Any process that modulates the frequency, rate or extent of wax biosynthetic process. Subtypes: GO:1904277, GO:1904278 References: PMID:24692420 Sources: GOC:TermGenie, GO_REF:0000058 Relationships: is a type of regulation of lipid biosynthetic process [GO:0046890]; regulates wax biosynthetic process [GO:0010025] Also known as: regulation of wax anabolism, regulation of wax biosynthesis, regulation of wax formation, regulation of wax synthesis